phosphoenolpyruvate-dependent sugar phosphotransferase system [GO:0009401] (biological process) Relationships: is a type of carbohydrate import across plasma membrane [GO:0098704] Also known as: PTS system References: PMID:31209249, PMID:33820910 Subtypes: phosphoenolpyruvate-dependent mannosylglycerate phosphotransferase system [GO:0051476] Definition: The uptake and phosphorylation of specific carbohydrates from the extracellular environment; uptake and phosphorylation are coupled, making the PTS a link between the uptake and metabolism of sugars; phosphoenolpyruvate is the original phosphate donor; phosphoenolpyruvate passes the phosphate via a signal transduction pathway, to enzyme 1 (E1), which in turn passes it on to the histidine protein, HPr; the next step in the system involves sugar-specific membrane-bound complex, enzyme 2 (EII), which transports the sugar into the cell; it includes the sugar permease, which catalyzes the transport reactions; EII is usually divided into three different domains, EIIA, EIIB, and EIIC.